{
  "term_id": "GO:0016323",
  "gene_symbol": "MTTP",
  "gene_name": "Microsomal triglyceride transfer protein large subunit",
  "term_label": "basolateral plasma membrane",
  "gene": "UniProtKB:P55157"
}